{
  "gene_name": "Pogo transposable element with ZNF domain",
  "gene_symbol": "POGZ",
  "term_label": "nucleus",
  "term_id": "GO:0005634",
  "gene": "UniProtKB:Q7Z3K3"
}